{
  "term_id": "GO:0002939",
  "gene_symbol": "TRMT10B",
  "gene_name": "tRNA methyltransferase 10 homolog B",
  "term_label": "tRNA N1-guanine methylation",
  "gene": "UniProtKB:Q6PF06"
}